{
  "term_id": "GO:0005634",
  "gene_symbol": "RALYL",
  "gene_name": "RNA-binding Raly-like protein",
  "term_label": "nucleus",
  "gene": "UniProtKB:Q86SE5"
}